{
  "term_label": "maintenance of presynaptic active zone structure",
  "gene": "UniProtKB:Q8IUD2",
  "gene_symbol": "ERC1",
  "gene_name": "ELKS_Rab6-interacting_CAST family member 1",
  "term_id": "GO:0048790"
}